galactose metabolic process [GO:0006012] (biological process) Also known as: galactose metabolism Subtypes: galactose catabolic process [GO:0019388], galactose biosynthetic process [GO:0046369] Sources: ISBN:0198506732 Definition: The chemical reactions and pathways involving galactose, the aldohexose galacto-hexose. D-galactose is widely distributed in combined form in plants, animals and microorganisms as a constituent of oligo- and polysaccharides; it also occurs in galactolipids and as its glucoside in lactose and melibiose. Relationships: is a type of hexose metabolic process [GO:0019318]